{
  "gene_symbol": "MAPK1",
  "gene": "UniProtKB:P28482",
  "term_id": "GO:0005737",
  "gene_name": "Mitogen-activated protein kinase 1",
  "term_label": "cytoplasm"
}